{
  "gene_name": "Beta-defensin 132",
  "term_id": "UNKNOWN:0001",
  "gene_symbol": "DEFB132",
  "gene": "UniProtKB:Q7Z7B7",
  "term_label": "Unknown molecular function"
}